mannosyltransferase complex [GO:0031501] (cellular component) Sources: GOC:mah Definition: A complex that possesses mannosyltransferase activity. Subtypes: GO:0000136, dolichyl-phosphate-mannose-protein mannosyltransferase complex [GO:0031502], dolichol-phosphate-mannose synthase complex [GO:0033185], glycosylphosphatidylinositol-mannosyltransferase II complex [GO:0120097], glycosylphosphatidylinositol-mannosyltransferase I complex [GO:1990529] Relationships: is a type of intracellular protein-containing complex [GO:0140535]; is a type of transferase complex [GO:1990234]